{
  "gene_symbol": "ATAD2",
  "gene_name": "ATPase family AAA domain-containing protein 2",
  "term_label": "nucleus",
  "term_id": "GO:0005634",
  "gene": "UniProtKB:Q6PL18"
}